{
  "term_id": "GO:0006357",
  "gene": "UniProtKB:A8MW92",
  "gene_name": "PHD finger protein 20-like protein 1",
  "gene_symbol": "PHF20L1",
  "term_label": "regulation of transcription by RNA polymerase II"
}